carnitine O-palmitoyltransferase activity [GO:0004095] (molecular function) Definition: Catalysis of the reaction: palmitoyl-CoA + L-carnitine = CoA + L-palmitoylcarnitine. Also known as: CPT, CPT I (outer membrane carnitine palmitoyl transferase), CPT-A, CPT-B, CPTi, CPTo, L-carnitine palmitoyltransferase activity, acylcarnitine transferase activity, carnitine palmitoyltransferase I, carnitine palmitoyltransferase II, carnitine palmitoyltransferase activity, carnitine palmitoyltransferase-A, outer malonyl-CoA inhibitable carnitine palmitoyltransferase activity, palmitoyl-CoA:L-carnitine O-palmitoyltransferase activity, palmitoylcarnitine transferase activity Sources: EC:2.3.1.21 Relationships: is a type of carnitine O-acyltransferase activity [GO:0016406]; is a type of O-palmitoyltransferase activity [GO:0016416]